negative regulation of cell cycle G1/S phase transition [GO:1902807] (biological process) Subtypes: negative regulation of G1/S transition of mitotic cell cycle [GO:2000134] Relationships: is a type of GO:1901988; is a type of regulation of cell cycle G1/S phase transition [GO:1902806]; negatively regulates cell cycle G1/S phase transition [GO:0044843] Definition: Any signaling pathway that decreases or inhibits the activity of a cell cycle cyclin-dependent protein kinase to modulate the switch from G1 phase to S phase of the cell cycle. Also known as: down regulation of cell cycle G1/S phase transition, down-regulation of cell cycle G1/S phase transition, downregulation of cell cycle G1/S phase transition, inhibition of cell cycle G1/S phase transition Sources: GOC:TermGenie, GOC:mtg_cell_cycle, GO_REF:0000058